{
  "gene_name": "Cytoplasmic aconitate hydratase",
  "gene": "UniProtKB:P21399",
  "term_label": "mitochondrion",
  "term_id": "GO:0005739",
  "gene_symbol": "ACO1"
}